{
  "gene_name": "Endothelial zinc finger protein induced by tumor necrosis factor alpha",
  "term_label": "nucleus",
  "gene_symbol": "ZNF71",
  "gene": "UniProtKB:Q9NQZ8",
  "term_id": "GO:0005634"
}